{
  "gene_name": "Sterile alpha motif domain-containing protein 14",
  "term_id": "GO:0051015",
  "term_label": "actin filament binding",
  "gene": "UniProtKB:Q8IZD0",
  "gene_symbol": "SAMD14"
}